{
  "gene_name": "Taste receptor type 2 member 20",
  "gene_symbol": "TAS2R20",
  "term_label": "Unknown molecular function",
  "gene": "UniProtKB:P59543",
  "term_id": "UNKNOWN:0001"
}